{
  "gene_name": "Gap junction beta-4 protein",
  "term_id": "GO:0005243",
  "gene": "UniProtKB:Q9NTQ9",
  "term_label": "gap junction channel activity",
  "gene_symbol": "GJB4"
}